{
  "gene_name": "Protein 4.2",
  "gene": "UniProtKB:P16452",
  "term_label": "Unknown cellular component",
  "term_id": "UNKNOWN:0003",
  "gene_symbol": "EPB42"
}